{
  "gene": "UniProtKB:Q15034",
  "gene_symbol": "HERC3",
  "gene_name": "Probable E3 ubiquitin-protein ligase HERC3",
  "term_id": "GO:0061630",
  "term_label": "ubiquitin protein ligase activity"
}